{
  "term_label": "cytoplasm",
  "gene_name": "C-Jun-amino-terminal kinase-interacting protein 4",
  "term_id": "GO:0005737",
  "gene": "UniProtKB:O60271",
  "gene_symbol": "SPAG9"
}